S-adenosylmethionine cycle [GO:0033353] (biological process) Sources: GOC:mah, MetaCyc:PWY-5041 Definition: A cyclic series of interconversions involving S-adenosylmethionine, S-adenosyl-L-homocysteine, L-cysteine, and L-methionine. Couples utilization of the methyl group of SAM with recycling of the homocysteinyl group and regeneration of methionine. Relationships: is a type of S-adenosylmethionine metabolic process [GO:0046500]; has part S-adenosylmethionine-homocysteine S-methyltransferase activity [GO:0008898] Also known as: SAM cycle, activated methyl cycle